{
  "gene": "UniProtKB:P15391",
  "term_label": "B cell receptor signaling pathway",
  "term_id": "GO:0050853",
  "gene_symbol": "CD19",
  "gene_name": "B-lymphocyte antigen CD19"
}